{
  "gene_name": "Myelin-associated glycoprotein",
  "term_label": "sialic acid binding",
  "gene_symbol": "MAG",
  "term_id": "GO:0033691",
  "gene": "UniProtKB:P20916"
}